{
  "gene": "UniProtKB:O75122",
  "gene_symbol": "CLASP2",
  "term_id": "GO:0005815",
  "term_label": "microtubule organizing center",
  "gene_name": "CLIP-associating protein 2"
}